{
  "term_label": "Unknown molecular function",
  "gene_symbol": "ATP6V1G2",
  "term_id": "UNKNOWN:0001",
  "gene": "UniProtKB:O95670",
  "gene_name": "V-type proton ATPase subunit G 2"
}